{
  "gene_symbol": "TMEM164",
  "gene_name": "Transmembrane protein 164",
  "term_id": "GO:0160020",
  "term_label": "positive regulation of ferroptosis",
  "gene": "UniProtKB:Q5U3C3"
}